nephrocyte differentiation [GO:0061319] (biological process) References: PMID:19783135 Sources: CL:0002520, GOC:dph, GOC:mtg_kidney_jan10 Relationships: is a type of renal filtration cell differentiation [GO:0061318] Definition: The process in which a relatively unspecialized cell acquires the specialized structural and/or functional features of a nephrocyte. A nephrocyte is an insect renal cell that filters hemolymph. Differentiation includes the processes involved in commitment of a cell to a specific fate and its subsequent development to the mature state. Subtypes: pericardial nephrocyte differentiation [GO:0061320], garland nephrocyte differentiation [GO:0061321], disseminated nephrocyte differentiation [GO:0061322]